biosynthetic process of antibacterial peptides active against Gram-positive bacteria [GO:0002815] (BP) Relationships: is a type of antibacterial peptide biosynthetic process [GO:0002780]; is part of defense response to Gram-positive bacterium [GO:0050830] Definition: The chemical reactions and pathways resulting in the formation of an antibacterial peptide with activity against Gram-positive bacteria. Regulation: regulated by regulation of biosynthetic process of antibacterial peptides active against Gram-positive bacteria [GO:0002816]; negatively regulated by negative regulation of biosynthetic process of antibacterial peptides active against Gram-positive bacteria [GO:0002817]; positively regulated by positive regulation of biosynthetic process of antibacterial peptides active against Gram-positive bacteria [GO:0006965] Sources: GOC:add